protein localization to postsynapse [GO:0062237] (BP) Definition: Any process in which a protein is transported to, and/or maintained at the postsynapse, the part of a synapse that is part of the post-synaptic cell. Subtypes: GO:1903539 Relationships: is a type of GO:0035418 References: PMID:31189538